{
  "gene_symbol": "ARL5B",
  "gene": "UniProtKB:Q96KC2",
  "gene_name": "ADP-ribosylation factor-like protein 5B",
  "term_id": "GO:0005802",
  "term_label": "trans-Golgi network"
}